{
  "term_label": "Golgi membrane",
  "gene": "UniProtKB:Q6UWH6",
  "gene_name": "Protein TEX261",
  "gene_symbol": "TEX261",
  "term_id": "GO:0000139"
}